{
  "gene_symbol": "ZKSCAN8P1",
  "gene_name": "HCG1646484",
  "gene": "UniProtKB:A0A8I5KTY6",
  "term_id": "UNKNOWN:0002",
  "term_label": "Unknown biological process"
}